{
  "gene": "UniProtKB:P25686",
  "term_id": "GO:0042026",
  "gene_symbol": "DNAJB2",
  "term_label": "protein refolding",
  "gene_name": "DnaJ homolog subfamily B member 2"
}